{
  "term_id": "UNKNOWN:0001",
  "gene_symbol": "SOWAHA",
  "gene_name": "Ankyrin repeat domain-containing protein SOWAHA",
  "gene": "UniProtKB:Q2M3V2",
  "term_label": "Unknown molecular function"
}